{
  "gene_name": "Protein O-mannosyl-transferase TMTC4",
  "term_id": "GO:0005783",
  "term_label": "endoplasmic reticulum",
  "gene": "UniProtKB:Q5T4D3",
  "gene_symbol": "TMTC4"
}